{
  "term_id": "UNKNOWN:0002",
  "gene": "UniProtKB:Q6GV28",
  "term_label": "Unknown biological process",
  "gene_symbol": "TMEM225",
  "gene_name": "Transmembrane protein 225"
}